eriodictyol 3'-O-methyltransferase activity [GO:0102761] (molecular function) Sources: RHEA:60948 Definition: Catalysis of the reaction: (S)-eriodictyol + S-adenosyl-L-methionine = (S)-homoeriodictyol + H+ + S-adenosyl-L-homocysteine. Relationships: is a type of methyltransferase activity [GO:0008168]